{
  "term_id": "UNKNOWN:0003",
  "gene_symbol": "CABP5",
  "term_label": "Unknown cellular component",
  "gene_name": "Calcium-binding protein 5",
  "gene": "UniProtKB:Q9NP86"
}